{
  "term_label": "mitochondrion organization",
  "gene_name": "Prohibitin-2",
  "gene_symbol": "PHB2",
  "gene": "UniProtKB:Q99623",
  "term_id": "GO:0007005"
}